cardioblast cell fate determination [GO:0007510] (biological process) Definition: The cell fate determination process in which a cell becomes capable of differentiating autonomously into a cardioblast cell regardless of its environment; upon determination, the cell fate cannot be reversed. A cardioblast is a cardiac precursor cell. It is a cell that has been committed to a cardiac fate, but will undergo more cell division rather than terminally differentiating. Sources: GOC:go_curators Relationships: is a type of GO:0060913; is part of cardioblast cell fate commitment [GO:0042684]